{
  "gene": "UniProtKB:Q96JE9",
  "gene_symbol": "MAP6",
  "gene_name": "Microtubule-associated protein 6",
  "term_label": "positive regulation of axonogenesis",
  "term_id": "GO:0050772"
}